{
  "gene_symbol": "CXCL16",
  "gene_name": "C-X-C motif chemokine 16",
  "gene": "UniProtKB:Q9H2A7",
  "term_label": "low-density lipoprotein particle receptor activity",
  "term_id": "GO:0005041"
}